{
  "gene_name": "Probable tRNA (uracil-O(2)-)-methyltransferase",
  "gene_symbol": "TRMT44",
  "term_id": "GO:0030488",
  "gene": "UniProtKB:Q8IYL2",
  "term_label": "tRNA methylation"
}